detection of auxin stimulus [GO:0009721] (biological process) Relationships: is a type of detection of hormone stimulus [GO:0009720]; is a type of response to auxin [GO:0009733] Definition: The series of events in which an auxin stimulus is received by a cell and converted into a molecular signal. Sources: GOC:sm Also known as: perception of auxin stimulus